{
  "term_label": "calcium-dependent phospholipase A2 activity",
  "gene_name": "Putative inactive group IIC secretory phospholipase A2",
  "term_id": "GO:0047498",
  "gene_symbol": "PLA2G2C",
  "gene": "UniProtKB:Q5R387"
}